{
  "term_id": "UNKNOWN:0002",
  "term_label": "Unknown biological process",
  "gene_symbol": "RBP3",
  "gene": "UniProtKB:P10745",
  "gene_name": "Retinol-binding protein 3"
}